mitochondrial mRNA editing complex [GO:0031019] (CC) Also known as: mitochondrial editosome Definition: An mRNA editing complex found in the mitochondrion. The best characterized example is that of Trypanosoma brucei, which catalyzes the insertion and deletion of uridylates. References: PMID:12139607 Sources: GOC:mah Relationships: is a type of mRNA editing complex [GO:0045293]; is_a GO:0098798